{
  "term_label": "immunoglobulin complex",
  "term_id": "GO:0019814",
  "gene_symbol": "IGLV5-52",
  "gene": "UniProtKB:A0A0A0MRZ9",
  "gene_name": "Immunoglobulin lambda variable 5-52"
}